{
  "term_label": "adherens junction",
  "gene_name": "Cadherin-13",
  "gene_symbol": "CDH13",
  "term_id": "GO:0005912",
  "gene": "UniProtKB:P55290"
}